positive regulation of skeletal muscle satellite cell proliferation [GO:1902724] (biological process) Definition: Any process that activates or increases the frequency, rate or extent of skeletal muscle satellite cell proliferation. Subtypes: positive regulation of growth factor dependent skeletal muscle satellite cell proliferation [GO:1902728] References: PMID:23212449 Sources: GOC:TermGenie, GO_REF:0000058 Relationships: is a type of regulation of skeletal muscle satellite cell proliferation [GO:0014842]; is a type of GO:0014858; positively regulates GO:0014841 Also known as: up regulation of satellite cell proliferation, up-regulation of satellite cell proliferation, upregulation of satellite cell proliferation, activation of satellite cell proliferation